{
  "gene_name": "MAP7 domain-containing protein 3",
  "gene_symbol": "MAP7D3",
  "term_label": "microtubule cytoskeleton organization",
  "gene": "UniProtKB:Q8IWC1",
  "term_id": "GO:0000226"
}